{
  "term_label": "heart development",
  "gene_symbol": "TGFB3",
  "gene_name": "Transforming growth factor beta-3 proprotein",
  "gene": "UniProtKB:P10600",
  "term_id": "GO:0007507"
}